{
  "term_id": "GO:0008360",
  "gene_name": "Plexin-B2",
  "gene": "UniProtKB:O15031",
  "term_label": "regulation of cell shape",
  "gene_symbol": "PLXNB2"
}